{
  "gene_symbol": "CHD6",
  "gene": "UniProtKB:Q8TD26",
  "gene_name": "Chromodomain-helicase-DNA-binding protein 6",
  "term_id": "GO:0006338",
  "term_label": "chromatin remodeling"
}